{
  "term_label": "Unknown cellular component",
  "gene": "UniProtKB:Q6ZUT9",
  "gene_name": "DENN domain-containing protein 5B",
  "gene_symbol": "DENND5B",
  "term_id": "UNKNOWN:0003"
}